cell adhesion mediated by integrin [GO:0033627] (biological process) Regulation: regulated by GO:0033628; negatively regulated by negative regulation of cell adhesion mediated by integrin [GO:0033629]; positively regulated by GO:0033630 Relationships: is a type of cell adhesion [GO:0007155] Also known as: cell adhesion mediated by integrin complex Definition: The attachment of a cell, either to another cell or to an underlying substrate such as the extracellular matrix, via an integrin, a heterodimeric adhesion receptor formed by the non-covalent association of particular alpha and beta subunits. Subtypes: cell-cell adhesion mediated by integrin [GO:0033631] References: PMID:12213832, PMID:14754902 Sources: GOC:add